{
  "gene_name": "G-protein coupled receptor 61",
  "gene": "UniProtKB:Q9BZJ8",
  "term_id": "GO:0043235",
  "term_label": "receptor complex",
  "gene_symbol": "GPR61"
}